{
  "term_label": "ubiquitin protein ligase binding",
  "gene": "UniProtKB:Q9GZQ8",
  "term_id": "GO:0031625",
  "gene_symbol": "MAP1LC3B",
  "gene_name": "Microtubule-associated proteins 1A_1B light chain 3B"
}